{
  "gene_symbol": "SERPINE3",
  "gene": "UniProtKB:A8MV23",
  "term_id": "GO:0005615",
  "gene_name": "Serpin E3",
  "term_label": "extracellular space"
}